Arp2/3 complex-mediated actin nucleation [GO:0034314] (biological process) Relationships: is a type of actin nucleation [GO:0045010] Definition: The actin nucleation process in which actin monomers combine to form a new branch on the side of an existing actin filament; mediated by the Arp2/3 protein complex and its interaction with other proteins. Regulation: RO_0002211 by regulation of Arp2/3 complex-mediated actin nucleation [GO:0034315]; negatively regulated by GO:0034316; positively regulated by positive regulation of Arp2/3 complex-mediated actin nucleation [GO:2000601] References: PMID:16959963, PMID:18640983 Sources: GOC:mah Also known as: actin filament branch nucleation, branched actin filament nucleation